{
  "gene_name": "Putative uncharacterized protein ENSP00000382790",
  "gene": "UniProtKB:A8MVM7",
  "gene_symbol": "A8MVM7",
  "term_label": "Unknown biological process",
  "term_id": "UNKNOWN:0002"
}